monoatomic anion transport [GO:0006820] (biological process) Sources: GOC:ai Also known as: anion transport Relationships: is a type of monoatomic ion transport [GO:0006811] Regulation: regulated by regulation of monoatomic anion transport [GO:0044070]; negatively regulated by negative regulation of monoatomic anion transport [GO:1903792]; positively regulated by positive regulation of monoatomic anion transport [GO:1903793] Definition: The directed movement of a monoatomic anion, into, out of or within a cell, or between cells, by means of some agent such as a transporter or pore. Monatomic anions (also called simple anions) are negatively charged ions consisting of exactly one atom. Subtypes: GO:0006821, iodide transport [GO:0015705], monoatomic anion transmembrane transport [GO:0098656]